{
  "gene": "UniProtKB:Q9BYR7",
  "gene_symbol": "KRTAP3-2",
  "term_label": "Unknown molecular function",
  "term_id": "UNKNOWN:0001",
  "gene_name": "Keratin-associated protein 3-2"
}